tyrosine ammonia-lyase activity [GO:0052883] (molecular function) Relationships: is a type of GO:0016841 Definition: Catalysis of the reaction: L-tyrosine = NH4 + trans-4-coumarate. Also known as: TAL activity, tyrase activity, L-tyrosine ammonia-lyase activity Sources: RHEA:24906